{
  "term_id": "GO:0005634",
  "gene_name": "Cyclic AMP-responsive element-binding protein 3-like protein 3",
  "gene": "UniProtKB:Q68CJ9",
  "term_label": "nucleus",
  "gene_symbol": "CREB3L3"
}